{
  "term_id": "UNKNOWN:0002",
  "term_label": "Unknown biological process",
  "gene_symbol": "KRTAP24-1",
  "gene_name": "Keratin-associated protein 24-1",
  "gene": "UniProtKB:Q3LI83"
}